propane 1,3-diol transport [GO:0015799] (biological process) Definition: The directed movement of 1,3-propanediol into, out of or within a cell, or between cells, by means of some agent such as a transporter or pore. Propanediol is a sweet colorless, viscous, hygroscopic liquid used as an antifreeze and in brake fluid; it is also as a humectant in cosmetics and personal care items, although it can be absorbed through the skin with harmful effects. Relationships: is a type of organic hydroxy compound transport [GO:0015850] References: PMID:24002752 Also known as: 1,3-propanediol transport